{
  "gene": "UniProtKB:Q9P2M1",
  "term_label": "Unknown molecular function",
  "gene_symbol": "LRP2BP",
  "term_id": "UNKNOWN:0001",
  "gene_name": "LRP2-binding protein"
}